{
  "term_id": "UNKNOWN:0003",
  "gene": "UniProtKB:P0C7V0",
  "gene_name": "Putative uncharacterized protein encoded by LINC00271",
  "term_label": "Unknown cellular component",
  "gene_symbol": "AHI1-DT"
}